{
  "term_label": "mitotic DNA replication initiation",
  "gene_symbol": "MCM3",
  "term_id": "GO:1902975",
  "gene": "UniProtKB:P25205",
  "gene_name": "DNA replication licensing factor MCM3"
}